negative regulation of secondary growth [GO:2000604] (BP) Definition: Any process that stops, prevents or reduces the frequency, rate or extent of secondary growth. Relationships: is a type of GO:0045926; is a type of regulation of secondary growth [GO:2000603]; negatively regulates secondary growth [GO:0080117] Sources: GOC:obol